{
  "gene_name": "Alkaline ceramidase 1",
  "term_id": "GO:0046514",
  "gene_symbol": "ACER1",
  "term_label": "ceramide catabolic process",
  "gene": "UniProtKB:Q8TDN7"
}